{
  "gene_symbol": "INSR",
  "gene_name": "Insulin receptor",
  "gene": "UniProtKB:P06213",
  "term_label": "insulin receptor signaling pathway",
  "term_id": "GO:0008286"
}